{
  "gene": "UniProtKB:Q6JVE9",
  "term_label": "Unknown cellular component",
  "gene_symbol": "LCN8",
  "term_id": "UNKNOWN:0003",
  "gene_name": "Epididymal-specific lipocalin-8"
}